{
  "gene_symbol": "CPA3",
  "term_label": "extracellular space",
  "gene_name": "Mast cell carboxypeptidase A",
  "gene": "UniProtKB:P15088",
  "term_id": "GO:0005615"
}